structural constituent of postsynaptic density [GO:0098919] (molecular function) Definition: The action of a molecule that contributes to the structural integrity of a postsynaptic density. Sources: GOC:dos Relationships: is a type of GO:0098879; is part of maintenance of postsynaptic density structure [GO:0099562]; occurs in postsynaptic density [GO:0014069]